{
  "gene_symbol": "PMS2P1",
  "gene_name": "Putative postmeiotic segregation increased 2-like protein 1",
  "gene": "UniProtKB:A4D2B8",
  "term_label": "Unknown molecular function",
  "term_id": "UNKNOWN:0001"
}